{
  "gene_name": "Dual specificity protein phosphatase 3",
  "term_id": "GO:0008138",
  "gene_symbol": "DUSP3",
  "term_label": "protein tyrosine/serine/threonine phosphatase activity",
  "gene": "UniProtKB:P51452"
}